{
  "term_label": "Unknown cellular component",
  "term_id": "UNKNOWN:0003",
  "gene_name": "E3 ubiquitin-protein ligase RNF170",
  "gene_symbol": "RNF170",
  "gene": "UniProtKB:Q96K19"
}